type I interferon receptor complex [GO:0038197] (cellular component) Relationships: is a type of GO:0098802 Definition: A heterodimeric protein complex that binds a type I interferon and transmits the signal across the membrane into the cell. Consists of an alpha subunit (IFNAR1) and a beta subunit (IFNAR2). References: PMID:17502368 Sources: GOC:cjm, GOC:signaling Also known as: interferon-alpha/beta receptor complex